{
  "gene_symbol": "BLZF1",
  "gene": "UniProtKB:Q9H2G9",
  "term_id": "GO:0043001",
  "term_label": "Golgi to plasma membrane protein transport",
  "gene_name": "Golgin-45"
}